middle lamella [GO:0009519] (CC) Sources: ISBN:0471245208 Definition: Layer of intercellular material, chiefly pectic substances, cementing together the primary walls of contiguous cells. Relationships: is a type of GO:0140047